chlorite O2-lyase activity [GO:0050587] (molecular function) Also known as: chloride:oxygen oxidoreductase activity, chlorite dismutase activity Sources: EC:1.13.11.49, RHEA:21404 Relationships: is a type of GO:0016702 Definition: Catalysis of the reaction: chloride + O2 = chlorite.